{
  "gene_symbol": "CCN4",
  "term_id": "GO:0007165",
  "gene_name": "CCN family member 4",
  "gene": "UniProtKB:O95388",
  "term_label": "signal transduction"
}